{
  "gene_symbol": "CDH13",
  "gene": "UniProtKB:P55290",
  "term_id": "GO:0045296",
  "gene_name": "Cadherin-13",
  "term_label": "cadherin binding"
}